{
  "term_id": "GO:0000812",
  "term_label": "Swr1 complex",
  "gene": "UniProtKB:Q9GZN1",
  "gene_name": "Actin-related protein 6",
  "gene_symbol": "ACTR6"
}